{
  "gene_name": "Leucine-rich repeat-containing protein 30",
  "term_id": "GO:0035556",
  "term_label": "intracellular signal transduction",
  "gene": "UniProtKB:A6NM36",
  "gene_symbol": "LRRC30"
}